{
  "term_label": "4 iron, 4 sulfur cluster binding",
  "gene_symbol": "RSAD2",
  "gene_name": "S-adenosylmethionine-dependent nucleotide dehydratase RSAD2",
  "gene": "UniProtKB:Q8WXG1",
  "term_id": "GO:0051539"
}